{
  "gene": "UniProtKB:Q8IUD6",
  "term_id": "GO:0004842",
  "term_label": "ubiquitin-protein transferase activity",
  "gene_name": "E3 ubiquitin-protein ligase RNF135",
  "gene_symbol": "RNF135"
}